{
  "gene_symbol": "STK16",
  "gene_name": "Serine_threonine-protein kinase 16",
  "gene": "UniProtKB:O75716",
  "term_id": "GO:0005794",
  "term_label": "Golgi apparatus"
}